{
  "term_label": "cell-matrix adhesion",
  "gene_symbol": "FERMT3",
  "gene": "UniProtKB:Q86UX7",
  "gene_name": "Fermitin family homolog 3",
  "term_id": "GO:0007160"
}